response to L-dopa [GO:1904473] (BP) Relationships: is a type of response to amino acid [GO:0043200]; is a type of response to oxygen-containing compound [GO:1901700]; is a type of response to L-phenylalanine derivative [GO:1904386] Subtypes: cellular response to L-dopa [GO:1904474] References: PMID:25044243 Sources: GOC:TermGenie, GO_REF:0000071 Definition: Any process that results in a change in state or activity of a cell or an organism (in terms of movement, secretion, enzyme production, gene expression, etc.) as a result of a L-dopa stimulus.